{
  "gene_name": "Coiled-coil domain-containing protein 62",
  "term_id": "GO:0030374",
  "gene_symbol": "CCDC62",
  "term_label": "obsolete nuclear receptor coactivator activity",
  "gene": "UniProtKB:Q6P9F0"
}